{
  "gene_symbol": "PURG",
  "term_label": "regulation of transcription by RNA polymerase II",
  "gene_name": "Purine-rich element-binding protein gamma",
  "gene": "UniProtKB:Q9UJV8",
  "term_id": "GO:0006357"
}